heart jogging [GO:0003146] (biological process) Also known as: cardiac jogging Definition: The morphogenetic process in which the heart cone is displaced to the left with respect to the vector of the anterior-posterior axis. Relationships: is a type of GO:0003143; is part of determination of heart left/right asymmetry [GO:0061371] References: PMID:9334285 Sources: GOC:mtg_heart